cell trailing edge membrane [GO:0031257] (CC) Definition: The portion of the plasma membrane surrounding the trailing edge of a motile cell. Sources: GOC:mah Also known as: trailing edge membrane Relationships: is a type of cellular anatomical structure [GO:0110165]; is part of GO:0005886; is part of GO:0031254 Subtypes: uropod membrane [GO:0031259]